{
  "term_label": "plasma membrane",
  "term_id": "GO:0005886",
  "gene_name": "Long-chain-fatty-acid--CoA ligase 4",
  "gene_symbol": "ACSL4",
  "gene": "UniProtKB:O60488"
}